{
  "gene_name": "Rho-related GTP-binding protein RhoG",
  "gene_symbol": "RHOG",
  "term_label": "GTPase activity",
  "gene": "UniProtKB:P84095",
  "term_id": "GO:0003924"
}